cellular response to adenine starvation [GO:0036223] (biological process) Relationships: is a type of cellular response to starvation [GO:0009267] Also known as: cellular response to adenine deprivation Definition: Any process that results in a change in state or activity of a cell (in terms of movement, secretion, enzyme production, gene expression, etc.) as a result of deprivation of adenine. Sources: GOC:ai